{
  "gene_symbol": "SUSD4",
  "term_id": "UNKNOWN:0002",
  "term_label": "Unknown biological process",
  "gene": "UniProtKB:Q5VX71",
  "gene_name": "Sushi domain-containing protein 4"
}